regulation of ribonucleoprotein complex localization [GO:2000197] (biological process) Subtypes: regulation of mRNA export from nucleus [GO:0010793], GO:2000198, positive regulation of ribonucleoprotein complex localization [GO:2000199], regulation of ribosomal subunit export from nucleus [GO:2000200], GO:2000238 Relationships: is a type of regulation of cellular localization [GO:0060341]; regulates GO:0071166 Definition: Any process that modulates the frequency, rate or extent of ribonucleoprotein complex localization. Also known as: regulation of RNP localization, regulation of cellular ribonucleoprotein complex localization, regulation of establishment and maintenance of ribonucleoprotein complex localization, regulation of ribonucleoprotein complex localisation Sources: GOC:mah